regulation of lung blood pressure [GO:0014916] (biological process) Also known as: regulation of pulmonary blood pressure Sources: GOC:mtg_cardio Relationships: is_a regulation of blood pressure [GO:0008217] Subtypes: positive regulation of lung blood pressure [GO:0061766], negative regulation of lung blood pressure [GO:0061767] Definition: The process that modulates the force with which blood travels through the lungs. The process is controlled by a balance of processes that increase pressure and decrease pressure.